2-deoxystreptamine N-acetyl-D-glucosaminyltransferase activity [GO:0102319] (molecular function) Sources: EC:2.4.1.283, GOC:pz Definition: Catalysis of the reaction: 2-deoxystreptamine(2+) + UDP-N-acetyl-alpha-D-glucosamine = H+ + 2'-N-acetylparomamine(2+) + UDP(3-). Relationships: is a type of hexosyltransferase activity [GO:0016758]